{
  "term_label": "positive regulation of cell migration",
  "gene_symbol": "KIT",
  "gene": "UniProtKB:P10721",
  "gene_name": "Mast_stem cell growth factor receptor Kit",
  "term_id": "GO:0030335"
}